{
  "gene_name": "Adenosylhomocysteinase",
  "term_label": "S-adenosylmethionine cycle",
  "gene": "UniProtKB:P23526",
  "term_id": "GO:0033353",
  "gene_symbol": "AHCY"
}